cortisol biosynthetic process [GO:0034651] (biological process) Relationships: is a type of glucocorticoid biosynthetic process [GO:0006704]; is_a GO:0034309; is a type of cortisol metabolic process [GO:0034650]; is_a ketone biosynthetic process [GO:0042181]; is a type of GO:0120255; is a type of tertiary alcohol biosynthetic process [GO:1902645] Definition: The chemical reactions and pathways resulting in the formation of cortisol, the steroid hormone 11-beta-17,21-trihydroxypregn-4-ene-3,20-dione. Cortisol is synthesized from cholesterol in the adrenal gland and controls carbohydrate, fat and protein metabolism and has anti-inflammatory properties. Also known as: cortisol biosynthesis, cortisol formation, cortisol synthesis, cortisol anabolism Regulation: RO_0002211 by regulation of cortisol biosynthetic process [GO:2000064]; negatively regulated by negative regulation of cortisol biosynthetic process [GO:2000065]; RO_0002213 by positive regulation of cortisol biosynthetic process [GO:2000066] Sources: GOC:BHF, GOC:mah, GOC:rl